{
  "gene_name": "Somatoliberin",
  "term_id": "GO:0005184",
  "gene": "UniProtKB:P01286",
  "term_label": "neuropeptide hormone activity",
  "gene_symbol": "GHRH"
}